{
  "gene_name": "Prenylcysteine oxidase 1",
  "gene_symbol": "PCYOX1",
  "gene": "UniProtKB:Q9UHG3",
  "term_id": "GO:0030327",
  "term_label": "prenylated protein catabolic process"
}